{
  "term_label": "ESCRT III complex",
  "gene": "UniProtKB:Q96FZ7",
  "term_id": "GO:0000815",
  "gene_symbol": "CHMP6",
  "gene_name": "Charged multivesicular body protein 6"
}